thrombocyte differentiation [GO:0002574] (biological process) Note: Note that platelets are the non-nucleated mammalian functional equivalent of the nucleated thrombocytes of non-mammalian vertebrates and are sometimes also referred to as thrombocytes. Platelet formation in mammals is covered by the biological_process term platelet formation ; GO:0030220. Definition: The process in which a relatively unspecialized myeloid precursor cell acquires the specialized features of a thrombocyte, a nucleated cell found in all vertebrates but mammals involved in hemostasis. Relationships: is a type of GO:0030099 Sources: GOC:add